{
  "term_id": "GO:0071577",
  "gene": "UniProtKB:Q9BRY0",
  "gene_symbol": "SLC39A3",
  "gene_name": "Zinc transporter ZIP3",
  "term_label": "zinc ion transmembrane transport"
}